{
  "term_label": "membrane",
  "gene_name": "Calcium_manganese antiporter SLC30A10",
  "term_id": "GO:0016020",
  "gene": "UniProtKB:Q6XR72",
  "gene_symbol": "SLC30A10"
}